{
  "term_id": "GO:0045104",
  "gene_symbol": "PPL",
  "gene_name": "Periplakin",
  "gene": "UniProtKB:O60437",
  "term_label": "intermediate filament cytoskeleton organization"
}